Rab GDP-dissociation inhibitor activity [GO:0005093] (molecular function) Relationships: is a type of GO:0005092 Definition: Prevents the dissociation of GDP from the small GTPase Rab, thereby preventing GTP from binding. Sources: GOC:mah